{
  "gene": "UniProtKB:P12830",
  "term_label": "adherens junction organization",
  "term_id": "GO:0034332",
  "gene_name": "Cadherin-1",
  "gene_symbol": "CDH1"
}